{
  "gene_name": "Fibroblast growth factor receptor 1",
  "term_label": "fibroblast growth factor receptor activity",
  "gene": "UniProtKB:P11362",
  "term_id": "GO:0005007",
  "gene_symbol": "FGFR1"
}